8-oxo-(d)RTP hydrolase activity [GO:0106379] (molecular function) Definition: Catalysis of the reaction: 8-oxo-(d)RTP + H20 = 8-oxo-(d)RMP + diphosphate + H+. References: PMID:11139615 Relationships: is a type of GO:0047429